{
  "gene_symbol": "HOXB4",
  "term_id": "GO:0000981",
  "gene_name": "Homeobox protein Hox-B4",
  "gene": "UniProtKB:P17483",
  "term_label": "DNA-binding transcription factor activity, RNA polymerase II-specific"
}